{
  "term_id": "GO:0005765",
  "gene": "UniProtKB:Q8IUH8",
  "gene_name": "Signal peptide peptidase-like 2C",
  "term_label": "lysosomal membrane",
  "gene_symbol": "SPPL2C"
}